{
  "term_label": "unfolded protein binding",
  "gene_symbol": "NUDCD3",
  "gene": "UniProtKB:Q8IVD9",
  "term_id": "GO:0051082",
  "gene_name": "NudC domain-containing protein 3"
}